{
  "gene_name": "Renal cancer differentiation gene 1 protein",
  "term_id": "UNKNOWN:0003",
  "gene_symbol": "C4orf46",
  "gene": "UniProtKB:Q504U0",
  "term_label": "Unknown cellular component"
}